{
  "gene_name": "Cilia- and flagella-associated protein 68",
  "gene_symbol": "CFAP68",
  "gene": "UniProtKB:Q9H5F2",
  "term_label": "Unknown biological process",
  "term_id": "UNKNOWN:0002"
}